{
  "gene_symbol": "MCM3",
  "gene": "UniProtKB:P25205",
  "term_label": "MCM complex",
  "gene_name": "DNA replication licensing factor MCM3",
  "term_id": "GO:0042555"
}